{
  "term_id": "UNKNOWN:0002",
  "gene": "UniProtKB:Q5JSS6",
  "term_label": "Unknown biological process",
  "gene_symbol": "MEIG1",
  "gene_name": "Meiosis expressed gene 1 protein homolog"
}